{
  "term_label": "membrane",
  "gene_symbol": "AKAP1",
  "gene_name": "A-kinase anchor protein 1, mitochondrial",
  "term_id": "GO:0016020",
  "gene": "UniProtKB:Q92667"
}